{
  "gene_symbol": "TOP1MT",
  "gene_name": "DNA topoisomerase I, mitochondrial",
  "term_label": "mitochondrial nucleoid",
  "gene": "UniProtKB:Q969P6",
  "term_id": "GO:0042645"
}